{
  "term_id": "UNKNOWN:0002",
  "gene": "UniProtKB:Q9Y6G5",
  "gene_name": "COMM domain-containing protein 10",
  "term_label": "Unknown biological process",
  "gene_symbol": "COMMD10"
}